G protein-coupled UDP receptor activity [GO:0045029] (molecular function) Relationships: is_a G protein-coupled pyrimidinergic nucleotide receptor activity [GO:0071553] Sources: GOC:mah Also known as: UDP-activated nucleotide receptor activity Definition: Combining with a nucleotide and transmitting the signal to a heterotrimeric G-protein complex to initiate a change in cell activity, activated by UDP.